3-hydroxybutyryl-CoA thiolase activity [GO:0018712] (molecular function) Definition: Catalysis of the reaction: 3-hydroxy-5-oxohexanoyl-CoA + CoASH = 3-hydroxybutyryl-CoA + acetyl-CoA. Sources: UM-BBD_reactionID:r0010 Relationships: is a type of acyltransferase activity, transferring groups other than amino-acyl groups [GO:0016747]